regulation of tRNA stability [GO:0036415] (biological process) References: PMID:21502523, PMID:23572593 Sources: GOC:aa Relationships: is a type of regulation of RNA stability [GO:0043487]; is_a regulation of tRNA catabolic process [GO:1902370] Subtypes: GO:0036416, GO:0036417 Definition: Any process that modulates the propensity of transfer RNA (tRNA) molecules to degradation. Includes processes that both stabilize and destabilize tRNAs.